{
  "term_id": "GO:0001671",
  "gene_name": "DnaJ homolog subfamily C member 24",
  "gene_symbol": "DNAJC24",
  "term_label": "ATPase activator activity",
  "gene": "UniProtKB:Q6P3W2"
}